trochlear nerve formation [GO:0021642] (biological process) Relationships: is a type of cranial nerve formation [GO:0021603]; is part of trochlear nerve morphogenesis [GO:0021639] Also known as: CN IV biosynthesis, CN IV formation Definition: The process that gives rise to the trochlear nerve. This process pertains to the initial formation of a structure from unspecified parts. The trochlear nerve is a motor nerve and is the only cranial nerve to exit the brain dorsally. The trochlear nerve innervates the superior oblique muscle. Sources: GOC:cls, GOC:dgh, GOC:dph, GOC:jid, GO_REF:0000021